{
  "term_label": "Unknown molecular function",
  "term_id": "UNKNOWN:0001",
  "gene_name": "Keratin, type I cytoskeletal 18",
  "gene": "UniProtKB:P05783",
  "gene_symbol": "KRT18"
}